cortisol sulfotransferase activity [GO:0047785] (molecular function) Also known as: glucocorticosteroid sulfotransferase activity, cortisol sulphotransferase activity, 3'-phosphoadenylyl-sulfate:cortisol 21-sulfotransferase activity, glucocorticoid sulfotransferase activity Sources: EC:2.8.2.18, RHEA:11884 Definition: Catalysis of the reaction: 3'-phospho-5'-adenylyl sulfate + cortisol = adenosine 3',5'-diphosphate + cortisol 21-sulfate + H+. Relationships: is a type of GO:0008146